{
  "gene": "UniProtKB:Q9Y615",
  "gene_symbol": "ACTL7A",
  "term_label": "cytoplasm",
  "term_id": "GO:0005737",
  "gene_name": "Actin-like protein 7A"
}